3-methyl-5-hydroxy-6-(3-carboxy-3-oxopropenyl)-1H-2-pyridon hydratase-aldolase activity [GO:0018815] (molecular function) Sources: MetaCyc:RXN-645, UM-BBD_reactionID:r0051 Relationships: is a type of hydro-lyase activity [GO:0016836] Definition: Catalysis of the reaction: 3-methyl-5-hydroxy-6-(3-carboxy-3-oxopropenyl)-1H-2-pyridon + H2O = 2-oxobut-3-enanoate + 2,5,6-trihydroxy-3-methylpyridine.